{
  "gene_name": "Unconventional myosin-Ie",
  "gene": "UniProtKB:Q12965",
  "gene_symbol": "MYO1E",
  "term_label": "cytoplasm",
  "term_id": "GO:0005737"
}